{
  "gene_name": "Probable lysine-specific demethylase 4F",
  "gene": "UniProtKB:A0A1W2PPD8",
  "term_label": "histone H3K9 demethylase activity",
  "term_id": "GO:0032454",
  "gene_symbol": "KDM4F"
}